{
  "gene": "UniProtKB:Q96CS4",
  "gene_name": "Zinc finger protein 689",
  "gene_symbol": "ZNF689",
  "term_label": "regulation of transcription by RNA polymerase II",
  "term_id": "GO:0006357"
}